{
  "term_id": "UNKNOWN:0002",
  "gene": "UniProtKB:Q96MR6",
  "gene_symbol": "CFAP57",
  "gene_name": "Cilia- and flagella-associated protein 57",
  "term_label": "Unknown biological process"
}